ADP-riboxanase activity [GO:0140740] (molecular function) Note: Note that this activity has two steps: a transfer of an ADP-ribose group, followed by the elimination of an ammonia group. Relationships: is a type of transferase activity, transferring phosphorus-containing groups [GO:0016772]; is a type of ammonia-lyase activity [GO:0016841]; is_a GO:0140096 Definition: Catalysis of the reaction: L-arginyl-[protein] + NAD+ = ADP-riboxanated L-argininyl-[protein] + H+ + NH4(+) + nicotinamide. References: PMID:34671164 Sources: RHEA:69500